{
  "gene_name": "Thyroid adenoma-associated protein",
  "gene": "UniProtKB:Q6YHU6",
  "gene_symbol": "THADA",
  "term_id": "GO:0030234",
  "term_label": "enzyme regulator activity"
}